{
  "term_label": "double-strand break repair via nonhomologous end joining",
  "term_id": "GO:0006303",
  "gene_symbol": "CYREN",
  "gene": "UniProtKB:Q9BWK5",
  "gene_name": "Cell cycle regulator of non-homologous end joining"
}